{
  "term_id": "UNKNOWN:0003",
  "gene_symbol": "POLR3K",
  "gene": "UniProtKB:Q9Y2Y1",
  "term_label": "Unknown cellular component",
  "gene_name": "DNA-directed RNA polymerase III subunit RPC10"
}